{
  "gene": "UniProtKB:A5D8T8",
  "term_label": "Unknown biological process",
  "gene_name": "C-type lectin domain family 18 member A",
  "gene_symbol": "CLEC18A",
  "term_id": "UNKNOWN:0002"
}